{
  "gene": "UniProtKB:Q7Z6J4",
  "gene_symbol": "FGD2",
  "gene_name": "FYVE, RhoGEF and PH domain-containing protein 2",
  "term_id": "GO:0005737",
  "term_label": "cytoplasm"
}